{
  "term_label": "Unknown cellular component",
  "term_id": "UNKNOWN:0003",
  "gene_symbol": "LINC01546",
  "gene_name": "Putative uncharacterized protein encoded by LINC01546",
  "gene": "UniProtKB:A6NGU7"
}